{
  "gene_name": "Dynamin-2",
  "term_label": "synapse",
  "gene": "UniProtKB:P50570",
  "term_id": "GO:0045202",
  "gene_symbol": "DNM2"
}